{
  "gene_name": "Cysteine-rich secretory protein LCCL domain-containing 1",
  "gene": "UniProtKB:Q9H336",
  "term_id": "UNKNOWN:0001",
  "gene_symbol": "CRISPLD1",
  "term_label": "Unknown molecular function"
}